{
  "gene_name": "Exosome complex component RRP4",
  "term_id": "GO:0003723",
  "gene_symbol": "EXOSC2",
  "gene": "UniProtKB:Q13868",
  "term_label": "RNA binding"
}